{
  "gene": "UniProtKB:P15509",
  "term_label": "peptide hormone binding",
  "gene_name": "Granulocyte-macrophage colony-stimulating factor receptor subunit alpha",
  "term_id": "GO:0017046",
  "gene_symbol": "CSF2RA"
}